{
  "gene": "UniProtKB:Q8N4S0",
  "gene_name": "Coiled-coil domain-containing protein 82",
  "term_id": "UNKNOWN:0002",
  "gene_symbol": "CCDC82",
  "term_label": "Unknown biological process"
}